dTTP catabolic process [GO:0046076] (biological process) Relationships: is a type of pyrimidine deoxyribonucleoside triphosphate catabolic process [GO:0009213]; is a type of pyrimidine deoxyribonucleotide catabolic process [GO:0009223]; is a type of dTTP metabolic process [GO:0046075] Definition: The chemical reactions and pathways resulting in the breakdown of dTTP, deoxyribosylthymine triphosphate. Sources: GOC:go_curators Also known as: dTTP breakdown, dTTP catabolism, dTTP degradation